{
  "gene": "UniProtKB:Q92813",
  "gene_symbol": "DIO2",
  "gene_name": "Type II iodothyronine deiodinase",
  "term_id": "UNKNOWN:0003",
  "term_label": "Unknown cellular component"
}